{
  "gene_symbol": "CATSPERB",
  "term_label": "cilium",
  "gene": "UniProtKB:Q9H7T0",
  "gene_name": "Cation channel sperm-associated auxiliary subunit beta",
  "term_id": "GO:0005929"
}